mitochondrial arginyl-tRNA aminoacylation [GO:0070144] (BP) Relationships: is a type of arginyl-tRNA aminoacylation [GO:0006420]; is a type of tRNA aminoacylation for mitochondrial protein translation [GO:0070127] Sources: GOC:mah, GOC:mcc Definition: The process of coupling arginine to arginyl-tRNA in a mitochondrion, catalyzed by arginyl-tRNA synthetase. In tRNA aminoacylation, the amino acid is first activated by linkage to AMP and then transferred to either the 2'- or the 3'-hydroxyl group of the 3'-adenosine residue of the tRNA.